{
  "term_label": "ubiquitin-like ligase-substrate adaptor activity",
  "gene_symbol": "KLHL26",
  "term_id": "GO:1990756",
  "gene_name": "Kelch-like protein 26",
  "gene": "UniProtKB:Q53HC5"
}